{
  "term_label": "regulation of transcription by RNA polymerase II",
  "gene_symbol": "FBXL19",
  "term_id": "GO:0006357",
  "gene": "UniProtKB:Q6PCT2",
  "gene_name": "F-box_LRR-repeat protein 19"
}